{
  "term_label": "dipeptidyl-peptidase activity",
  "gene_name": "Lysosomal Pro-X carboxypeptidase",
  "gene_symbol": "PRCP",
  "term_id": "GO:0008239",
  "gene": "UniProtKB:P42785"
}